{
  "gene_symbol": "CHMP5",
  "term_label": "nuclear envelope",
  "term_id": "GO:0005635",
  "gene": "UniProtKB:Q9NZZ3",
  "gene_name": "Charged multivesicular body protein 5"
}